{
  "gene_name": "Partitioning defective 3 homolog",
  "gene_symbol": "PARD3",
  "gene": "UniProtKB:Q8TEW0",
  "term_id": "GO:0045197",
  "term_label": "establishment or maintenance of epithelial cell apical/basal polarity"
}